{
  "term_label": "ABC-type sterol transporter activity",
  "gene_name": "ATP-binding cassette sub-family G member 1",
  "gene_symbol": "ABCG1",
  "term_id": "GO:0034041",
  "gene": "UniProtKB:P45844"
}